{
  "term_id": "GO:0038023",
  "term_label": "signaling receptor activity",
  "gene_symbol": "TLR6",
  "gene": "UniProtKB:Q9Y2C9",
  "gene_name": "Toll-like receptor 6"
}